{
  "gene_symbol": "ZSWIM1",
  "term_id": "UNKNOWN:0002",
  "gene_name": "Zinc finger SWIM domain-containing protein 1",
  "term_label": "Unknown biological process",
  "gene": "UniProtKB:Q9BR11"
}